{
  "gene_symbol": "SRM",
  "gene": "UniProtKB:P19623",
  "term_id": "GO:0005829",
  "gene_name": "Spermidine synthase",
  "term_label": "cytosol"
}